{
  "term_id": "GO:0005634",
  "gene_symbol": "DDX17",
  "gene": "UniProtKB:Q92841",
  "term_label": "nucleus",
  "gene_name": "Probable ATP-dependent RNA helicase DDX17"
}